{
  "term_id": "GO:0007189",
  "gene": "UniProtKB:P22888",
  "gene_name": "Lutropin-choriogonadotropic hormone receptor",
  "term_label": "adenylate cyclase-activating G protein-coupled receptor signaling pathway",
  "gene_symbol": "LHCGR"
}